opsonin receptor activity [GO:0001847] (molecular function) Sources: GOC:add, GOC:signaling, ISBN:0781735149 Relationships: is a type of transmembrane signaling receptor activity [GO:0004888]; has part opsonin binding [GO:0001846] Subtypes: complement component C1q receptor activity [GO:0001857], complement component iC3b receptor activity [GO:0001858], complement component C4b receptor activity [GO:0001861], collectin receptor activity [GO:0001863], GO:0004877, GO:0004878, GO:0008029 Definition: Combining with an opsonin and transmitting the signal from one side of the membrane to the other to initiate a change in cell activity.